oxidoreductase activity, acting on a heme group of donors [GO:0016675] (molecular function) Subtypes: cytochrome bo3 ubiquinol oxidase activity [GO:0009486], oxidoreductase activity, acting on a heme group of donors, nitrogenous group as acceptor [GO:0016677], iron-cytochrome-c reductase activity [GO:0047726], nitric oxide dioxygenase activity, heme protein as donor [GO:0141118] Sources: GOC:ai Relationships: is a type of GO:0016491 Also known as: oxidoreductase activity, acting on haem group of donors, oxidoreductase activity, acting on heme group of donors, other acceptors Definition: Catalysis of an oxidation-reduction (redox) reaction in which a heme group acts as a hydrogen or electron donor and reduces a hydrogen or electron acceptor.